{
  "gene": "UniProtKB:Q9BZV3",
  "term_id": "GO:0005540",
  "gene_symbol": "IMPG2",
  "term_label": "hyaluronic acid binding",
  "gene_name": "Interphotoreceptor matrix proteoglycan 2"
}